{
  "term_label": "Unknown cellular component",
  "gene": "UniProtKB:Q9BYQ3",
  "gene_symbol": "KRTAP9-3",
  "gene_name": "Keratin-associated protein 9-3",
  "term_id": "UNKNOWN:0003"
}